{
  "term_label": "Unknown cellular component",
  "gene_name": "Putative ankyrin repeat domain-containing protein 20A3",
  "gene": "UniProtKB:Q5VUR7",
  "gene_symbol": "ANKRD20A3P",
  "term_id": "UNKNOWN:0003"
}